{
  "gene_symbol": "STAT6",
  "gene_name": "Signal transducer and activator of transcription 6",
  "term_id": "GO:0007259",
  "gene": "UniProtKB:P42226",
  "term_label": "cell surface receptor signaling pathway via JAK-STAT"
}